{
  "term_id": "GO:0019731",
  "gene": "UniProtKB:Q8TCV5",
  "gene_name": "WAP four-disulfide core domain protein 5",
  "gene_symbol": "WFDC5",
  "term_label": "antibacterial humoral response"
}